{
  "gene_name": "Fibroblast growth factor 10",
  "term_id": "GO:0005615",
  "gene_symbol": "FGF10",
  "gene": "UniProtKB:O15520",
  "term_label": "extracellular space"
}